4-alpha-D-(1->4)-alpha-D-glucanotrehalose trehalohydrolase activity [GO:0033942] (molecular function) Sources: EC:3.2.1.141 Definition: Catalysis of the hydrolysis of alpha-(1->4)-D-glucosidic linkage in 4-alpha-D-{(1->4)-alpha-D-glucanosyl}n trehalose to yield trehalose and alpha-(1->4)-D-glucan. Also known as: 4-alpha-D-{(1,4)-alpha-D-glucano}trehalose glucanohydrolase (trehalose-producing) activity, 4-alpha-D-{(1->4)-alpha-D-glucano}trehalose glucanohydrolase (trehalose-producing) activity, malto-oligosyltrehalose trehalohydrolase activity, maltooligosyl trehalose trehalohydrolase activity Relationships: is a type of GO:0004553